{
  "term_id": "GO:0005615",
  "term_label": "extracellular space",
  "gene_name": "Reelin",
  "gene_symbol": "RELN",
  "gene": "UniProtKB:P78509"
}